{
  "gene_name": "Large ribosomal subunit protein uL30m",
  "term_id": "GO:0005739",
  "term_label": "mitochondrion",
  "gene_symbol": "MRPL30",
  "gene": "UniProtKB:Q8TCC3"
}